negative regulation of interferon-beta production [GO:0032688] (biological process) References: PMID:15546383 Sources: GOC:mah Relationships: is a type of negative regulation of type I interferon production [GO:0032480]; is a type of regulation of interferon-beta production [GO:0032648]; negatively regulates GO:0032608 Definition: Any process that stops, prevents, or reduces the frequency, rate, or extent of interferon-beta production. Also known as: down regulation of interferon-beta production, down-regulation of interferon-beta production, downregulation of interferon-beta production, negative regulation of IFN-beta production, inhibition of interferon-beta production, negative regulation of interferon-beta biosynthetic process, negative regulation of interferon-beta secretion